{
  "gene": "UniProtKB:Q9GZX7",
  "term_id": "GO:0000932",
  "gene_symbol": "AICDA",
  "gene_name": "Single-stranded DNA cytosine deaminase",
  "term_label": "P-body"
}